{
  "gene": "UniProtKB:O94760",
  "gene_symbol": "DDAH1",
  "gene_name": "N(G),N(G)-dimethylarginine dimethylaminohydrolase 1",
  "term_id": "GO:0000052",
  "term_label": "citrulline metabolic process"
}